{
  "gene": "UniProtKB:P14923",
  "gene_symbol": "JUP",
  "gene_name": "Junction plakoglobin",
  "term_label": "transcription coactivator activity",
  "term_id": "GO:0003713"
}